diphosphate hydrolysis-driven proton transmembrane transporter activity [GO:0009678] (MF) Relationships: is a type of proton transmembrane transporter activity [GO:0015078]; is a type of active monoatomic ion transmembrane transporter activity [GO:0022853]; has part GO:0004427 Sources: GOC:mtg_transport, Wikipedia:Proton-pumping_pyrophosphatase Also known as: PP(i) hydrolysis-driven proton transmembrane transporter activity, proton-translocating pyrophosphatase activity, H+-exporting diphosphatase, hydrogen-translocating pyrophosphatase activity, proton-pumping diphosphatase, proton-pumping pyrophosphatase, pyrophosphate hydrolysis-driven proton transmembrane transporter activity Definition: Catalysis of the reaction: diphosphate + H+(in) + H2O = 2 H+(out) + 2 phosphate.